{
  "gene_symbol": "NOTCH1",
  "gene": "UniProtKB:P46531",
  "gene_name": "Neurogenic locus notch homolog protein 1",
  "term_id": "GO:0007411",
  "term_label": "axon guidance"
}